{
  "gene": "UniProtKB:P60002",
  "term_id": "GO:0000993",
  "gene_name": "Transcription elongation factor 1 homolog",
  "term_label": "RNA polymerase II complex binding",
  "gene_symbol": "ELOF1"
}